trans-synaptic signaling by lipid [GO:0099541] (BP) Definition: Cell-cell signaling from post to pre-synapse, across the synaptic cleft, mediated by a lipid. Sources: GOC:dos Relationships: is a type of trans-synaptic signaling [GO:0099537] Subtypes: GO:0098920, GO:0099542, trans-synaptic signaling by lipid, modulating synaptic transmission [GO:0099552]